{
  "gene_name": "Zinc finger protein 512",
  "gene": "UniProtKB:Q96ME7",
  "gene_symbol": "ZNF512",
  "term_label": "Unknown cellular component",
  "term_id": "UNKNOWN:0003"
}